{
  "gene_symbol": "NCOA6",
  "gene_name": "Nuclear receptor coactivator 6",
  "term_label": "transcription coactivator activity",
  "term_id": "GO:0003713",
  "gene": "UniProtKB:Q14686"
}